{
  "gene_symbol": "COL12A1",
  "gene_name": "Collagen alpha-1(XII) chain",
  "term_label": "Unknown molecular function",
  "gene": "UniProtKB:Q99715",
  "term_id": "UNKNOWN:0001"
}